{
  "term_id": "GO:0010133",
  "term_label": "L-proline catabolic process to L-glutamate",
  "gene": "UniProtKB:Q9UF12",
  "gene_name": "Hydroxyproline dehydrogenase",
  "gene_symbol": "PRODH2"
}